{
  "term_id": "UNKNOWN:0002",
  "term_label": "Unknown biological process",
  "gene": "UniProtKB:A0A0J9YVP2",
  "gene_symbol": "IGHJ6",
  "gene_name": "Immunoglobulin heavy joining 6 (Fragment)"
}